{
  "gene_symbol": "RPL36AL",
  "gene_name": "Ribosomal protein eL42-like",
  "gene": "UniProtKB:Q969Q0",
  "term_label": "cytoplasmic translation",
  "term_id": "GO:0002181"
}